{
  "gene_symbol": "RAB11A",
  "gene": "UniProtKB:P62491",
  "term_id": "GO:0032402",
  "gene_name": "Ras-related protein Rab-11A",
  "term_label": "melanosome transport"
}